{
  "term_label": "calcium ion transmembrane transport",
  "gene": "UniProtKB:O60721",
  "gene_symbol": "SLC24A1",
  "gene_name": "Sodium_potassium_calcium exchanger 1",
  "term_id": "GO:0070588"
}